purine nucleotide metabolic process [GO:0006163] (biological process) Regulation: regulated by regulation of purine nucleotide metabolic process [GO:1900542]; negatively regulated by negative regulation of purine nucleotide metabolic process [GO:1900543]; positively regulated by GO:1900544 Definition: The chemical reactions and pathways involving a purine nucleotide, a compound consisting of nucleoside (a purine base linked to a deoxyribose or ribose sugar) esterified with a phosphate group at either the 3' or 5'-hydroxyl group of the sugar. Relationships: is a type of nucleotide metabolic process [GO:0009117]; is a type of GO:0072521 Sources: GOC:go_curators, ISBN:0198506732 Subtypes: purine nucleotide biosynthetic process [GO:0006164], purine nucleotide catabolic process [GO:0006195], GO:0006739, purine ribonucleotide metabolic process [GO:0009150], GO:0009151, purine nucleotide interconversion [GO:0015950], NAD+ metabolic process [GO:0019674], cyclic purine nucleotide metabolic process [GO:0052652] Also known as: purine nucleotide metabolism, purine metabolic process, purine metabolism